{
  "gene_name": "Signal-regulatory protein delta",
  "term_label": "Unknown biological process",
  "term_id": "UNKNOWN:0002",
  "gene": "UniProtKB:Q9H106",
  "gene_symbol": "SIRPD"
}